{
  "gene": "UniProtKB:Q9H3L0",
  "term_label": "cobalamin metabolic process",
  "term_id": "GO:0009235",
  "gene_name": "Cobalamin trafficking protein CblD",
  "gene_symbol": "MMADHC"
}